{
  "gene_name": "Putative C-type lectin-like domain family 1",
  "term_id": "UNKNOWN:0002",
  "gene_symbol": "CLECL1P",
  "gene": "UniProtKB:Q8IZS7",
  "term_label": "Unknown biological process"
}